primary oocyte stage [GO:0048159] (biological process) Definition: The stage in oogenesis when the oocyte has a nucleus slightly larger than those of the adjacent cells and is surrounded by a layer of loose squamous epithelial cells. Sources: GOC:jid, GOC:mtg_sensu, ISBN:0198542771 Relationships: is a type of mammalian oogenesis stage [GO:0022605] Also known as: mammalian oogenesis stage 2